avascular cornea development in camera-type eye [GO:0036331] (biological process) Definition: The progression of an avascular cornea over time, from its formation to the mature structure. Corneal avascularity (the absence of blood vessels in the cornea) is required for optical clarity and optimal vision. Avascular corneas are present in most animals, except Manatees. Also known as: avascular cornea development Relationships: is a type of cornea development in camera-type eye [GO:0061303] References: PMID:16849433, PMID:17051153 Sources: GOC:uh